{
  "gene_symbol": "IL4R",
  "gene": "UniProtKB:P24394",
  "gene_name": "Interleukin-4 receptor subunit alpha",
  "term_id": "GO:0004913",
  "term_label": "interleukin-4 receptor activity"
}